cerebellar stellate cell differentiation [GO:0021710] (biological process) Relationships: is a type of cell differentiation in hindbrain [GO:0021533]; is a type of central nervous system neuron differentiation [GO:0021953]; is part of GO:0021688 References: PMID:15157725 Sources: GOC:cls, GOC:dgh, GOC:dph, GOC:jid, GO_REF:0000021 Definition: The process in which neuroblasts acquire specialized structural and/or functional features that characterize the mature cerebellar stellate cell. Differentiation includes the processes involved in commitment of a neuroblast to a cerebellar stellate cell fate. A cerebellar stellate cell is an inhibitory GABAergic interneuron found in the cerebellar cortex.